{
  "gene": "UniProtKB:Q3ZCQ3",
  "term_id": "UNKNOWN:0003",
  "gene_name": "Membrane protein FAM174B",
  "term_label": "Unknown cellular component",
  "gene_symbol": "FAM174B"
}